{
  "term_id": "GO:0032580",
  "gene_name": "Golgin subfamily A member 8C",
  "gene_symbol": "GOLGA8CP",
  "gene": "UniProtKB:A6NN73",
  "term_label": "Golgi cisterna membrane"
}